medium-term memory [GO:0072375] (BP) Relationships: is a type of memory [GO:0007613] References: PMID:14659098, PMID:7923375 Sources: GOC:sart Also known as: middle-term memory, MTM Definition: The memory process that deals with the storage, retrieval and modification of information received at a time ago that is intermediate between that of short and long term memory (30min - 7hrs in Drosophila melanogaster).